negative regulation of cellular response to amino acid starvation [GO:1903574] (biological process) Definition: Any process that stops, prevents or reduces the frequency, rate or extent of a cellular response to amino acid starvation. Relationships: is_a negative regulation of response to nutrient levels [GO:0032108]; is a type of negative regulation of cellular process [GO:0048523]; is a type of regulation of cellular response to amino acid starvation [GO:1903832]; RO_0002212 cellular response to amino acid starvation [GO:0034198] References: PMID:11381086 Sources: GOC:PARL, GOC:TermGenie, GOC:bf, GO_REF:0000058 Also known as: down regulation of cellular response to amino acid starvation, down-regulation of cellular response to amino acid starvation, downregulation of cellular response to amino acid starvation, inhibition of cellular response to amino acid starvation